{
  "gene_symbol": "IQCA1",
  "gene": "UniProtKB:Q86XH1",
  "term_label": "microtubule severing ATPase activity",
  "gene_name": "Dynein regulatory complex protein 11",
  "term_id": "GO:0008568"
}